{
  "gene_name": "Immunoglobulin heavy variable 3-43D",
  "gene_symbol": "IGHV3-43D",
  "term_label": "immunoglobulin mediated immune response",
  "gene": "UniProtKB:P0DP04",
  "term_id": "GO:0016064"
}